negative regulation of cellular response to growth factor stimulus [GO:0090288] (biological process) Subtypes: negative regulation of BMP signaling pathway [GO:0030514], negative regulation of vascular endothelial growth factor receptor signaling pathway [GO:0030948], negative regulation of fibroblast growth factor receptor signaling pathway [GO:0040037], negative regulation of neurotrophin TRK receptor signaling pathway [GO:0051387], negative regulation of cellular response to vascular endothelial growth factor stimulus [GO:1902548], GO:1903845, GO:1904848, negative regulation of cellular response to hepatocyte growth factor stimulus [GO:2001113] Relationships: is a type of negative regulation of response to stimulus [GO:0048585]; is a type of regulation of cellular response to growth factor stimulus [GO:0090287]; negatively regulates cellular response to growth factor stimulus [GO:0071363] Definition: Any process that decreases the rate, frequency, or extent of a change in state or activity of a cell (in terms of movement, secretion, enzyme production, gene expression, etc.) as a result of a growth factor stimulus. Sources: GOC:BHF